{
  "gene_symbol": "APP",
  "term_label": "axonogenesis",
  "gene": "UniProtKB:P05067",
  "gene_name": "Amyloid-beta precursor protein",
  "term_id": "GO:0007409"
}